{
  "gene_name": "Axin-1",
  "term_id": "GO:0019901",
  "gene_symbol": "AXIN1",
  "gene": "UniProtKB:O15169",
  "term_label": "protein kinase binding"
}